{
  "term_id": "UNKNOWN:0001",
  "gene": "UniProtKB:A1L4Q6",
  "term_label": "Unknown molecular function",
  "gene_name": "Putative uncharacterized protein FLJ41423",
  "gene_symbol": "A1L4Q6"
}